{
  "gene_symbol": "CENPQ",
  "gene": "UniProtKB:Q7L2Z9",
  "term_label": "inner kinetochore",
  "term_id": "GO:0000939",
  "gene_name": "Centromere protein Q"
}